{
  "gene": "UniProtKB:P25440",
  "term_id": "GO:0006338",
  "term_label": "chromatin remodeling",
  "gene_symbol": "BRD2",
  "gene_name": "Bromodomain-containing protein 2"
}